{
  "gene_name": "Immunoglobulin subtype domain-containing protein",
  "term_id": "GO:0002767",
  "term_label": "immune response-inhibiting cell surface receptor signaling pathway",
  "gene_symbol": "A0A5F9Z9Y6",
  "gene": "UniProtKB:A0A5F9Z9Y6"
}